{
  "gene_name": "Cell division cycle protein 16 homolog",
  "gene": "UniProtKB:Q13042",
  "term_label": "protein ubiquitination",
  "gene_symbol": "CDC16",
  "term_id": "GO:0016567"
}